{
  "gene": "UniProtKB:Q9BR39",
  "term_id": "GO:0005789",
  "gene_name": "Junctophilin-2",
  "gene_symbol": "JPH2",
  "term_label": "endoplasmic reticulum membrane"
}